{
  "term_id": "GO:0030280",
  "term_label": "structural constituent of skin epidermis",
  "gene": "UniProtKB:Q14533",
  "gene_symbol": "KRT81",
  "gene_name": "Keratin, type II cuticular Hb1"
}